beta-apiosyl-beta-glucosidase activity [GO:0033956] (molecular function) Definition: Catalysis of the reaction: 7-[beta-D-apiofuranosyl-(1->6)-beta-D-glucopyranosyloxy]isoflavonoid + H2O = a 7-hydroxyisoflavonoid + beta-D-apiofuranosyl-(1->6)-D-glucose. Also known as: 7-[beta-D-apiofuranosyl-(1->6)-beta-D-glucopyranosyloxy]isoflavonoid beta-D-apiofuranosyl-(1->6)-D-glucohydrolase activity, furcatin hydrolase activity, isoflavonoid 7-O-beta-apiosyl-glucoside beta-glucosidase activity, isoflavonoid-7-O-beta[D-apiosyl-(1->6)-beta-D-glucoside] disaccharidase activity Sources: EC:3.2.1.161 Relationships: is a type of beta-glucosidase activity [GO:0008422]